{
  "gene": "UniProtKB:P49459",
  "gene_name": "Ubiquitin-conjugating enzyme E2 A",
  "gene_symbol": "UBE2A",
  "term_id": "GO:0033503",
  "term_label": "HULC complex"
}